maintenance of meiotic sister chromatid cohesion [GO:0034090] (biological process) Sources: GOC:mah Relationships: is a type of maintenance of sister chromatid cohesion [GO:0034086]; is part of GO:0051177 Definition: The process in which the association between sister chromatids of a replicated chromosome is maintained as chromosomes condense, attach to the spindle in a bipolar orientation, and congress to the metaphase plate during a meiotic cell cycle. Regulation: regulated by GO:0034094; negatively regulated by negative regulation of maintenance of meiotic sister chromatid cohesion [GO:0034095]; positively regulated by positive regulation of maintenance of meiotic sister chromatid cohesion [GO:0034096] Subtypes: maintenance of meiotic sister chromatid cohesion, centromeric [GO:0035875]